{
  "gene_symbol": "SLAIN2",
  "term_label": "Unknown molecular function",
  "term_id": "UNKNOWN:0001",
  "gene": "UniProtKB:Q9P270",
  "gene_name": "SLAIN motif-containing protein 2"
}